antigen processing and presentation of endogenous peptide antigen via MHC class Ib via ER pathway, TAP-independent [GO:0002490] (biological process) Relationships: is_a GO:0002488 Definition: The process in which an antigen-presenting cell expresses a peptide antigen of endogenous origin on its cell surface in association with an MHC class Ib protein complex following intracellular transport via a pathway not requiring TAP (transporter associated with antigen processing). The peptide is typically a fragment of a larger endogenous protein which has been degraded within the cell. Class Ib here refers to non-classical class I molecules, such as those of the HLA-E gene family. References: PMID:15928678 Sources: GOC:add Also known as: TAP-independent antigen processing and presentation of endogenous peptide antigen via MHC class Ib via ER pathway, TAP-independent endogenous peptide antigen processing and presentation via MHC class Ib via ER pathway, endogenous peptide antigen processing and presentation via MHC class Ib via ER pathway, TAP-independent